{
  "gene_name": "DNA polymerase delta catalytic subunit",
  "gene_symbol": "POLD1",
  "gene": "UniProtKB:P28340",
  "term_label": "nucleotide-excision repair, DNA gap filling",
  "term_id": "GO:0006297"
}